{
  "gene_name": "Membrane-anchored junction protein",
  "gene": "UniProtKB:Q3KP22",
  "term_label": "homologous chromosome pairing at meiosis",
  "term_id": "GO:0007129",
  "gene_symbol": "MAJIN"
}